{
  "term_id": "GO:0007423",
  "gene": "UniProtKB:Q13516",
  "gene_name": "Oligodendrocyte transcription factor 2",
  "term_label": "sensory organ development",
  "gene_symbol": "OLIG2"
}